{
  "term_id": "GO:0051607",
  "gene_symbol": "APOBEC3B",
  "term_label": "defense response to virus",
  "gene": "UniProtKB:Q9UH17",
  "gene_name": "DNA dC-dU-editing enzyme APOBEC-3B"
}